{
  "term_label": "histone binding",
  "term_id": "GO:0042393",
  "gene_symbol": "HPF1",
  "gene_name": "Histone PARylation factor 1",
  "gene": "UniProtKB:Q9NWY4"
}